{
  "gene_name": "COUP transcription factor 2",
  "term_id": "UNKNOWN:0003",
  "gene": "UniProtKB:P24468",
  "gene_symbol": "NR2F2",
  "term_label": "Unknown cellular component"
}